{
  "gene_symbol": "TM9SF2",
  "gene_name": "Transmembrane 9 superfamily member 2",
  "term_id": "UNKNOWN:0001",
  "term_label": "Unknown molecular function",
  "gene": "UniProtKB:Q99805"
}